{
  "gene_symbol": "NHP2",
  "gene": "UniProtKB:Q9NX24",
  "gene_name": "H_ACA ribonucleoprotein complex subunit 2",
  "term_label": "box H/ACA snoRNA binding",
  "term_id": "GO:0034513"
}